positive regulation of ERK1 and ERK2 cascade [GO:0070374] (biological process) Definition: Any process that activates or increases the frequency, rate or extent of signal transduction mediated by the ERK1 and ERK2 cascade. Sources: GOC:mah Relationships: is a type of GO:0043410; is a type of regulation of ERK1 and ERK2 cascade [GO:0070372]; positively regulates ERK1 and ERK2 cascade [GO:0070371] Also known as: positive regulation of ERK cascade, positive regulation of ERK1 and ERK2 signaling pathway, positive regulation of ERK1 and ERK2 signalling pathway, positive regulation of ERK1/2 cascade, up regulation of ERK1 and ERK2 cascade, up-regulation of ERK1 and ERK2 cascade, upregulation of ERK1 and ERK2 cascade, activation of ERK1 and ERK2 cascade, positive regulation of ERK1 cascade, positive regulation of ERK2 cascade, positive regulation of MAPK1 cascade, positive regulation of MAPK3 cascade, stimulation of ERK1 and ERK2 cascade